{
  "term_label": "serine-type endopeptidase inhibitor activity",
  "gene_name": "Serpin B4",
  "gene_symbol": "SERPINB4",
  "gene": "UniProtKB:P48594",
  "term_id": "GO:0004867"
}